{
  "gene_name": "Lymphokine-activated killer T-cell-originated protein kinase",
  "term_id": "GO:0004674",
  "gene_symbol": "PBK",
  "term_label": "protein serine/threonine kinase activity",
  "gene": "UniProtKB:Q96KB5"
}